{
  "term_label": "Unknown biological process",
  "gene": "UniProtKB:A4D1U4",
  "gene_name": "DENN domain-containing protein 11",
  "gene_symbol": "DENND11",
  "term_id": "UNKNOWN:0002"
}